positive regulation of interleukin-10 production [GO:0032733] (biological process) Sources: GOC:mah Relationships: is a type of positive regulation of cytokine production [GO:0001819]; is a type of regulation of interleukin-10 production [GO:0032653]; positively regulates interleukin-10 production [GO:0032613] Definition: Any process that activates or increases the frequency, rate, or extent of interleukin-10 production. Also known as: positive regulation of IL-10 production, up regulation of interleukin-10 production, up-regulation of interleukin-10 production, upregulation of interleukin-10 production, activation of interleukin-10 production, positive regulation of interleukin-10 biosynthetic process, positive regulation of interleukin-10 secretion, stimulation of interleukin-10 production